{
  "term_id": "UNKNOWN:0003",
  "term_label": "Unknown cellular component",
  "gene": "UniProtKB:Q96NT3",
  "gene_symbol": "GUCD1",
  "gene_name": "Protein GUCD1"
}